{
  "term_id": "GO:0034272",
  "gene_name": "Beclin-2",
  "term_label": "phosphatidylinositol 3-kinase complex, class III, type II",
  "gene_symbol": "BECN2",
  "gene": "UniProtKB:A8MW95"
}